{
  "gene_name": "Serine_threonine-protein kinase TAO3",
  "gene": "UniProtKB:Q9H2K8",
  "gene_symbol": "TAOK3",
  "term_label": "regulation of MAPK cascade",
  "term_id": "GO:0043408"
}